{
  "term_label": "plasma membrane",
  "gene_name": "Rab3 GTPase-activating protein non-catalytic subunit",
  "term_id": "GO:0005886",
  "gene": "UniProtKB:Q9H2M9",
  "gene_symbol": "RAB3GAP2"
}